pentraxin binding [GO:0001864] (molecular function) Note: Note that pentraxins include such proteins as serum amyloid P component (SAP) and C-reactive protein (CRP). Relationships: is a type of opsonin binding [GO:0001846] Sources: GOC:add, ISBN:0781735149 Definition: Binding to a pentraxin, a member of a family of inflammatory proteins with a radially symmetric arrangement of five identical, noncovalently linked chains in a pentagonal array.